{
  "gene": "UniProtKB:Q9UGM1",
  "term_label": "neuron projection",
  "gene_symbol": "CHRNA9",
  "gene_name": "Neuronal acetylcholine receptor subunit alpha-9",
  "term_id": "GO:0043005"
}